{
  "term_id": "GO:0006955",
  "gene_symbol": "IGKV6-21",
  "term_label": "immune response",
  "gene_name": "Immunoglobulin kappa variable 6-21",
  "gene": "UniProtKB:A0A0C4DH24"
}